{
  "gene": "UniProtKB:P61158",
  "gene_name": "Actin-related protein 3",
  "gene_symbol": "ACTR3",
  "term_label": "Arp2/3 protein complex",
  "term_id": "GO:0005885"
}